{
  "gene_symbol": "AGR2",
  "gene_name": "Anterior gradient protein 2 homolog",
  "term_label": "dystroglycan binding",
  "gene": "UniProtKB:O95994",
  "term_id": "GO:0002162"
}